{
  "gene": "UniProtKB:Q99594",
  "term_id": "GO:0048568",
  "term_label": "embryonic organ development",
  "gene_name": "Transcriptional enhancer factor TEF-5",
  "gene_symbol": "TEAD3"
}